{
  "gene_name": "Flavin-containing monooxygenase 1",
  "gene_symbol": "FMO1",
  "term_label": "Unknown cellular component",
  "term_id": "UNKNOWN:0003",
  "gene": "UniProtKB:Q01740"
}